{
  "gene_symbol": "FIGLA",
  "gene": "UniProtKB:Q6QHK4",
  "term_label": "DNA-binding transcription factor activity, RNA polymerase II-specific",
  "gene_name": "Factor in the germline alpha",
  "term_id": "GO:0000981"
}